{
  "gene_name": "Spartin",
  "term_id": "UNKNOWN:0001",
  "term_label": "Unknown molecular function",
  "gene": "UniProtKB:Q8N0X7",
  "gene_symbol": "SPART"
}